protein phosphorylated amino acid binding [GO:0045309] (molecular function) Subtypes: phosphotyrosine residue binding [GO:0001784], GO:0050815, phosphothreonine residue binding [GO:0050816] Relationships: is a type of phosphoprotein binding [GO:0051219] Definition: Binding to a phosphorylated amino acid residue within a protein. Sources: GOC:go_curators Also known as: phosphoprotein amino acid binding